deoxyribose phosphate catabolic process [GO:0046386] (biological process) Also known as: deoxyribose phosphate breakdown, deoxyribose phosphate catabolism, deoxyribose phosphate degradation Definition: The chemical reactions and pathways resulting in the breakdown of deoxyribose phosphate, the phosphorylated sugar 2-deoxy-erythro-pentose. Relationships: is a type of GO:0006796; is a type of organophosphate catabolic process [GO:0046434]; is a type of carbohydrate derivative catabolic process [GO:1901136] Subtypes: GO:0006018, purine deoxyribonucleotide catabolic process [GO:0009155], GO:0009223 Sources: ISBN:0198506732